{
  "gene_symbol": "THRA",
  "term_label": "positive regulation of transcription by RNA polymerase II",
  "term_id": "GO:0045944",
  "gene": "UniProtKB:P10827",
  "gene_name": "Thyroid hormone receptor alpha"
}